{
  "gene_name": "Ubiquitin carboxyl-terminal hydrolase MINDY-3",
  "gene_symbol": "MINDY3",
  "term_label": "Unknown biological process",
  "gene": "UniProtKB:Q9H8M7",
  "term_id": "UNKNOWN:0002"
}